{
  "term_label": "RNA polymerase II cis-regulatory region sequence-specific DNA binding",
  "gene_symbol": "SP6",
  "gene": "UniProtKB:Q3SY56",
  "term_id": "GO:0000978",
  "gene_name": "Transcription factor Sp6"
}